beta-alanopine dehydrogenase activity [GO:0047697] (molecular function) Sources: EC:1.5.1.26, RHEA:21684 Also known as: b-alanopine dehydrogenase activity, N-(D-1-carboxyethyl)-beta-alanine:NAD+ oxidoreductase (beta-alanine-forming) Definition: Catalysis of the reaction: (R)-beta-alanopine + H2O + NAD+ = beta-alanine + H+ + NADH + pyruvate. Relationships: is_a oxidoreductase activity, acting on the CH-NH group of donors, NAD or NADP as acceptor [GO:0016646]